regulation of seed maturation [GO:2000034] (biological process) Definition: Any process that modulates the frequency, rate or extent of seed maturation. Relationships: is_a regulation of seed development [GO:0080050]; regulates seed maturation [GO:0010431] Sources: GOC:obol Subtypes: GO:2000033, negative regulation of seed maturation [GO:2000692], GO:2000693